{
  "gene": "UniProtKB:Q07001",
  "term_label": "synapse",
  "gene_name": "Acetylcholine receptor subunit delta",
  "term_id": "GO:0045202",
  "gene_symbol": "CHRND"
}